{
  "term_id": "GO:0004674",
  "gene": "UniProtKB:P19784",
  "gene_symbol": "CSNK2A2",
  "gene_name": "Casein kinase II subunit alpha'",
  "term_label": "protein serine/threonine kinase activity"
}